{
  "gene_name": "NK1 transcription factor-related protein 2",
  "gene_symbol": "NKX1-2",
  "gene": "UniProtKB:Q9UD57",
  "term_id": "GO:0000978",
  "term_label": "RNA polymerase II cis-regulatory region sequence-specific DNA binding"
}